{
  "term_label": "plasma membrane",
  "gene": "UniProtKB:O14863",
  "gene_name": "Probable proton-coupled zinc antiporter SLC30A4",
  "term_id": "GO:0005886",
  "gene_symbol": "SLC30A4"
}